{
  "gene_symbol": "LDLRAD1",
  "gene_name": "Low-density lipoprotein receptor class A domain-containing protein 1",
  "gene": "UniProtKB:Q5T700",
  "term_id": "UNKNOWN:0003",
  "term_label": "Unknown cellular component"
}